cell proliferation involved in pronephros development [GO:0039015] (biological process) Relationships: is a type of cell proliferation involved in kidney development [GO:0072111]; is part of GO:0048793 Sources: GOC:mtg_kidney_jan10 Definition: The multiplication or reproduction of cells, resulting in the expansion of the population in the pronephros. Also known as: cell proliferation involved in pronephric kidney development